{
  "gene_symbol": "SMPD4",
  "term_label": "glycerophospholipid catabolic process",
  "gene_name": "Sphingomyelin phosphodiesterase 4",
  "gene": "UniProtKB:Q9NXE4",
  "term_id": "GO:0046475"
}